{
  "term_label": "cysteine-type deubiquitinase activity",
  "term_id": "GO:0004843",
  "gene_name": "Ubiquitin carboxyl-terminal hydrolase isozyme L1",
  "gene_symbol": "UCHL1",
  "gene": "UniProtKB:P09936"
}